{
  "gene": "UniProtKB:Q9H299",
  "gene_symbol": "SH3BGRL3",
  "term_id": "GO:0005829",
  "term_label": "cytosol",
  "gene_name": "SH3 domain-binding glutamic acid-rich-like protein 3"
}